{
  "term_id": "GO:0019911",
  "gene_symbol": "GPM6B",
  "gene": "UniProtKB:Q13491",
  "term_label": "structural constituent of myelin sheath",
  "gene_name": "Neuronal membrane glycoprotein M6-b"
}